{
  "gene": "UniProtKB:O75110",
  "term_id": "GO:0005886",
  "gene_symbol": "ATP9A",
  "term_label": "plasma membrane",
  "gene_name": "Probable phospholipid-transporting ATPase IIA"
}